{
  "term_label": "cell surface receptor signaling pathway",
  "gene_name": "Pappalysin-2",
  "gene_symbol": "PAPPA2",
  "term_id": "GO:0007166",
  "gene": "UniProtKB:Q9BXP8"
}